cellular response to molecule of bacterial origin [GO:0071219] (biological process) Subtypes: cellular response to bacterial lipoprotein [GO:0071220], cellular response to lipopolysaccharide [GO:0071222], cellular response to lipoteichoic acid [GO:0071223], cellular response to peptidoglycan [GO:0071224] Relationships: is a type of response to molecule of bacterial origin [GO:0002237]; is a type of cellular response to biotic stimulus [GO:0071216] Definition: Any process that results in a change in state or activity of a cell (in terms of movement, secretion, enzyme production, gene expression, etc.) as a result of a stimulus by molecules of bacterial origin such as peptides derived from bacterial flagellin. Also known as: cellular response to bacteria associated molecule, cellular response to bacterial associated molecule, cellular response to bacterium associated molecule Sources: GOC:mah